{
  "gene": "UniProtKB:P49458",
  "term_id": "UNKNOWN:0001",
  "gene_name": "Signal recognition particle 9 kDa protein",
  "gene_symbol": "SRP9",
  "term_label": "Unknown molecular function"
}